dendritic cell proliferation [GO:0044565] (biological process) Definition: The expansion of a dendritic cell population by cell division. A dendritic cell is a cell of hematopoietic origin, typically resident in particular tissues, specialized in the uptake, processing, and transport of antigens to lymph nodes for the purpose of stimulating an immune response via T cell activation. References: PMID:18469816 Sources: CL:0000451 Relationships: is a type of mononuclear cell proliferation [GO:0032943]